{
  "term_id": "UNKNOWN:0002",
  "gene": "UniProtKB:Q4G148",
  "term_label": "Unknown biological process",
  "gene_name": "Glucoside xylosyltransferase 1",
  "gene_symbol": "GXYLT1"
}